{
  "gene_name": "Cerebral cavernous malformations 2 protein",
  "term_label": "Unknown cellular component",
  "gene": "UniProtKB:Q9BSQ5",
  "term_id": "UNKNOWN:0003",
  "gene_symbol": "CCM2"
}